{
  "term_label": "positive regulation of insulin receptor signaling pathway",
  "gene_symbol": "IGF2",
  "gene": "UniProtKB:P01344",
  "gene_name": "Insulin-like growth factor II",
  "term_id": "GO:0046628"
}